signal recognition particle, endoplasmic reticulum targeting [GO:0005786] (cellular component) Sources: GOC:mtg_sensu, ISBN:0198506732 Relationships: is a type of GO:0048500 Also known as: SRP, signal sequence receptor complex Definition: A ribonucleoprotein particle of 325 kDa composed of a 7S (300 nucleotide) RNA molecule and a complex of six different polypeptides. This binds both to the N-terminal signal peptide for proteins destined for the endoplasmic reticulum as they emerge from the large ribosomal subunit and also to the ribosome. This binding arrests further translation thereby preventing the proteins from being released into the cytosol. The SRP-ribosome complex then diffuses to the endoplasmic reticulum where it is bound to the signal recognition particle receptor, which allows resumption of protein synthesis and facilitates the passage of the growing polypeptide chain through the translocon. Through a process involving GTP hydrolysis, the SRP-SRP receptor complex dissociates and SRP returns to the cytosol. Of the six polypeptides of SRP the 54 kDa subunit (SRP54) is the central player. It contains an N-terminal GTPase domain and a C-terminal domain that binds directly to the signal peptide and the SRP RNA. Examples of this component are found in Mus musculus, Saccharomyces cerevisiae and Arabidopsis thaliana.